{
  "gene_name": "DNA-directed RNA polymerases I, II, and III subunit RPABC2",
  "term_label": "transcription by RNA polymerase II",
  "term_id": "GO:0006366",
  "gene": "UniProtKB:P61218",
  "gene_symbol": "POLR2F"
}